{
  "gene_name": "DNA topoisomerase 3-alpha",
  "gene_symbol": "TOP3A",
  "term_label": "DNA repair",
  "gene": "UniProtKB:Q13472",
  "term_id": "GO:0006281"
}